{
  "gene_symbol": "CACNA1A",
  "gene_name": "Voltage-dependent P_Q-type calcium channel subunit alpha-1A",
  "term_id": "GO:0008331",
  "gene": "UniProtKB:O00555",
  "term_label": "high voltage-gated calcium channel activity"
}